{
  "gene": "UniProtKB:P22415",
  "term_label": "regulation of transcription by RNA polymerase II",
  "gene_name": "Upstream stimulatory factor 1",
  "gene_symbol": "USF1",
  "term_id": "GO:0006357"
}